{
  "term_id": "GO:0070373",
  "term_label": "negative regulation of ERK1 and ERK2 cascade",
  "gene": "UniProtKB:Q7Z699",
  "gene_name": "Sprouty-related, EVH1 domain-containing protein 1",
  "gene_symbol": "SPRED1"
}